{
  "gene_name": "Serine_threonine-protein kinase 17B",
  "gene_symbol": "STK17B",
  "term_id": "GO:0004674",
  "gene": "UniProtKB:O94768",
  "term_label": "protein serine/threonine kinase activity"
}